lipooligosaccharide metabolic process [GO:1901269] (biological process) Relationships: is a type of carbohydrate derivative metabolic process [GO:1901135] Definition: The chemical reactions and pathways involving lipooligosaccharide. Subtypes: lipid A metabolic process [GO:0046493], GO:1901270, lipooligosaccharide biosynthetic process [GO:1901271] Sources: GOC:TermGenie, GOC:yaf, UniPathway:UPA00501 Also known as: lipooligosaccharide metabolism